{
  "term_label": "cytoplasm",
  "gene_name": "tRNA N6-adenosine threonylcarbamoyltransferase",
  "gene_symbol": "OSGEP",
  "term_id": "GO:0005737",
  "gene": "UniProtKB:Q9NPF4"
}